{
  "term_label": "cGMP catabolic process",
  "gene": "UniProtKB:O00408",
  "gene_name": "cGMP-dependent 3',5'-cyclic phosphodiesterase",
  "gene_symbol": "PDE2A",
  "term_id": "GO:0046069"
}